{
  "term_id": "GO:0006886",
  "term_label": "intracellular protein transport",
  "gene_symbol": "RAB29",
  "gene_name": "Ras-related protein Rab-7L1",
  "gene": "UniProtKB:O14966"
}